{
  "term_id": "GO:0009897",
  "gene_symbol": "PDCD1",
  "term_label": "external side of plasma membrane",
  "gene_name": "Programmed cell death protein 1",
  "gene": "UniProtKB:Q15116"
}